{
  "term_label": "cell differentiation",
  "term_id": "GO:0030154",
  "gene_name": "Homeobox protein Nkx-2.8",
  "gene": "UniProtKB:O15522",
  "gene_symbol": "NKX2-8"
}